{
  "gene_name": "Glucose-6-phosphatase 2",
  "gene_symbol": "G6PC2",
  "term_id": "GO:0006094",
  "term_label": "gluconeogenesis",
  "gene": "UniProtKB:Q9NQR9"
}